{
  "gene_symbol": "GDF5",
  "term_id": "GO:0030509",
  "gene": "UniProtKB:P43026",
  "gene_name": "Growth_differentiation factor 5",
  "term_label": "BMP signaling pathway"
}